{
  "gene_name": "Signal transducer and activator of transcription 4",
  "term_id": "GO:0006357",
  "gene_symbol": "STAT4",
  "gene": "UniProtKB:Q14765",
  "term_label": "regulation of transcription by RNA polymerase II"
}